{
  "gene_name": "Nuclear receptor subfamily 4 group A member 2",
  "gene_symbol": "NR4A2",
  "gene": "UniProtKB:P43354",
  "term_label": "nucleus",
  "term_id": "GO:0005634"
}